{
  "gene": "UniProtKB:A8MWL7",
  "term_id": "UNKNOWN:0001",
  "gene_symbol": "TMEM14DP",
  "term_label": "Unknown molecular function",
  "gene_name": "Transmembrane protein 14DP"
}